{
  "gene_symbol": "KLRC1",
  "gene": "UniProtKB:P26715",
  "gene_name": "NKG2-A_NKG2-B type II integral membrane protein",
  "term_id": "GO:0045954",
  "term_label": "positive regulation of natural killer cell mediated cytotoxicity"
}